{
  "term_label": "calcium-mediated signaling",
  "gene": "UniProtKB:Q9ULJ8",
  "gene_symbol": "PPP1R9A",
  "term_id": "GO:0019722",
  "gene_name": "Neurabin-1"
}